{
  "term_id": "GO:0030154",
  "gene": "UniProtKB:Q07869",
  "term_label": "cell differentiation",
  "gene_symbol": "PPARA",
  "gene_name": "Peroxisome proliferator-activated receptor alpha"
}